protein-glutaryllysine deglutarylase activity [GO:0061697] (molecular function) Relationships: is_a NAD-dependent protein lysine deacylase activity [GO:0141218] References: PMID:24703693 Sources: RHEA:47664 Note: This reaction is the removal of a glutaryl group from a glutarylated lysine residue of a protein or peptide. Definition: Catalysis of the reaction: N(6)-glutaryl-L-lysyl-[protein] + NAD+ + H2O = 2''-O-glutaryl-ADP-D-ribose + nicotinamide + L-lysyl-[protein].